{
  "gene_name": "D-amino-acid oxidase",
  "term_id": "GO:0036088",
  "gene": "UniProtKB:P14920",
  "gene_symbol": "DAO",
  "term_label": "D-serine catabolic process"
}